{
  "gene_symbol": "CCNG2",
  "gene": "UniProtKB:Q16589",
  "term_id": "GO:0000082",
  "term_label": "G1/S transition of mitotic cell cycle",
  "gene_name": "Cyclin-G2"
}